spindle pole body anchor activity [GO:0140475] (molecular function) References: PMID:19942852 Relationships: is a type of cytoskeletal anchor activity [GO:0008093] Definition: The binding activity of a protein that brings together the spindle pole body and one or more other molecules, permitting them to function in a coordinated way. Subtypes: spindle pole body-nuclear membrane anchor activity [GO:0106166]